{
  "gene_symbol": "NANOS3",
  "gene": "UniProtKB:P60323",
  "term_id": "GO:0017148",
  "term_label": "negative regulation of translation",
  "gene_name": "Nanos homolog 3"
}